{
  "term_label": "meiotic cell cycle",
  "gene_symbol": "TUBGCP5",
  "gene": "UniProtKB:Q96RT8",
  "term_id": "GO:0051321",
  "gene_name": "Gamma-tubulin complex component 5"
}